{
  "term_label": "hyaluronan biosynthetic process",
  "gene_name": "Hyaluronan synthase 3",
  "gene": "UniProtKB:O00219",
  "gene_symbol": "HAS3",
  "term_id": "GO:0030213"
}